{
  "gene_name": "Olfactory receptor 8J3",
  "term_label": "Unknown cellular component",
  "gene": "UniProtKB:Q8NGG0",
  "gene_symbol": "OR8J3",
  "term_id": "UNKNOWN:0003"
}